inhibitory MHC class Ib receptor activity [GO:0062080] (molecular function) Relationships: is a type of MHC class Ib receptor activity [GO:0032394] Subtypes: HLA-E specific inhibitory MHC class Ib receptor activity [GO:0062082], HLA-G specific inhibitory MHC class Ib receptor activity [GO:0062083] Sources: DOI:10.1002/9780470015902.a0024246 Definition: Combining with a MHC class Ib protein complex to mediate signaling that inhibits activation of a lymphocyte.